SUMO-targeted ubiquitin ligase complex [GO:0033768] (cellular component) Relationships: is a type of nuclear ubiquitin ligase complex [GO:0000152] References: PMID:17762864, PMID:17762865 Sources: GOC:vw Definition: A nuclear ubiquitin ligase complex that specifically targets SUMOylated proteins; the complex is formed of homodimers or heterodimers of RNF4 family ubiquitin ligases and is conserved in eukaryotes.